{
  "gene": "UniProtKB:A0A075B702",
  "gene_symbol": "TRAJ41",
  "term_id": "UNKNOWN:0002",
  "gene_name": "T cell receptor alpha joining 41 (Fragment)",
  "term_label": "Unknown biological process"
}